{
  "term_label": "reciprocal meiotic recombination",
  "gene_symbol": "DMC1",
  "gene_name": "Meiotic recombination protein DMC1_LIM15 homolog",
  "gene": "UniProtKB:Q14565",
  "term_id": "GO:0007131"
}